{
  "gene_name": "Fascin",
  "term_label": "lamellipodium",
  "gene": "UniProtKB:Q16658",
  "term_id": "GO:0030027",
  "gene_symbol": "FSCN1"
}